{
  "term_id": "GO:0009897",
  "gene_symbol": "CD4",
  "gene": "UniProtKB:P01730",
  "term_label": "external side of plasma membrane",
  "gene_name": "T-cell surface glycoprotein CD4"
}